{
  "gene": "UniProtKB:Q6IQ21",
  "term_label": "transcription cis-regulatory region binding",
  "term_id": "GO:0000976",
  "gene_symbol": "ZNF770",
  "gene_name": "Zinc finger protein 770"
}